{
  "term_id": "GO:0004325",
  "gene_symbol": "FECH",
  "term_label": "ferrochelatase activity",
  "gene": "UniProtKB:P22830",
  "gene_name": "Ferrochelatase, mitochondrial"
}